plastid small ribosomal subunit [GO:0000312] (cellular component) Sources: GOC:mcc Relationships: is a type of organellar small ribosomal subunit [GO:0000314]; is part of GO:0009547 Subtypes: chloroplast small ribosomal subunit [GO:0022629] Definition: The smaller of the two subunits of a plastid ribosome.